nucleotide-binding oligomerization domain containing 2 signaling pathway [GO:0070431] (biological process) Regulation: RO_0002211 by regulation of nucleotide-binding oligomerization domain containing 2 signaling pathway [GO:0070432]; negatively regulated by GO:0070433; positively regulated by GO:0070434 Relationships: is a type of nucleotide-binding domain, leucine rich repeat containing receptor signaling pathway [GO:0035872] References: PMID:17944960, PMID:18585455 Sources: GOC:add Also known as: NOD2 signaling pathway, nucleotide-binding oligomerization domain containing 2 signalling pathway Definition: The series of molecular signals initiated by the binding of a ligand (such as a bacterial peptidoglycan) to a cytoplasmic nucleotide-binding oligomerization domain containing 2 (NOD2) protein receptor, and ending with regulation of a downstream cellular process.